{
  "term_label": "T cell activation",
  "gene_name": "T-cell surface glycoprotein CD4",
  "term_id": "GO:0042110",
  "gene_symbol": "CD4",
  "gene": "UniProtKB:P01730"
}